{
  "gene": "UniProtKB:Q15773",
  "term_id": "GO:0005634",
  "term_label": "nucleus",
  "gene_symbol": "MLF2",
  "gene_name": "Myeloid leukemia factor 2"
}